{
  "gene_symbol": "CIAPIN1",
  "gene": "UniProtKB:Q6FI81",
  "gene_name": "Anamorsin",
  "term_label": "cytoplasm",
  "term_id": "GO:0005737"
}